{
  "gene_name": "Gamma-tubulin complex component 2",
  "term_label": "microtubule minus-end binding",
  "gene": "UniProtKB:Q9BSJ2",
  "term_id": "GO:0051011",
  "gene_symbol": "TUBGCP2"
}